{
  "term_label": "potassium channel activator activity",
  "term_id": "GO:0099104",
  "gene_name": "Leucine-rich repeat-containing protein 38",
  "gene": "UniProtKB:Q5VT99",
  "gene_symbol": "LRRC38"
}